{
  "gene_symbol": "TRAV12-3",
  "term_id": "UNKNOWN:0003",
  "term_label": "Unknown cellular component",
  "gene_name": "T cell receptor alpha variable 12-3",
  "gene": "UniProtKB:A0A0B4J271"
}